{
  "term_label": "endoplasmic reticulum",
  "gene_symbol": "TMEM247",
  "term_id": "GO:0005783",
  "gene": "UniProtKB:A6NEH6",
  "gene_name": "Transmembrane protein 247"
}